{
  "term_id": "UNKNOWN:0001",
  "gene": "UniProtKB:Q96N19",
  "gene_name": "Integral membrane protein GPR137",
  "gene_symbol": "GPR137",
  "term_label": "Unknown molecular function"
}